{
  "gene_name": "Uncharacterized protein",
  "gene_symbol": "LOC122539214",
  "term_id": "GO:0000978",
  "gene": "UniProtKB:A0A7P0TAN4",
  "term_label": "RNA polymerase II cis-regulatory region sequence-specific DNA binding"
}